{
  "gene_name": "Tyrosine-protein phosphatase non-receptor type 6",
  "gene": "UniProtKB:P29350",
  "term_id": "GO:0005737",
  "term_label": "cytoplasm",
  "gene_symbol": "PTPN6"
}